cellular response to chloroquine [GO:1902350] (biological process) Definition: Any process that results in a change in state or activity of a cell (in terms of movement, secretion, enzyme production, gene expression, etc.) as a result of a chloroquine stimulus. Relationships: is a type of cellular response to nitrogen compound [GO:1901699]; is_a response to chloroquine [GO:1902349] References: PMID:23922869 Sources: GOC:TermGenie, GOC:kmv